{
  "gene_symbol": "CAPN10",
  "gene": "UniProtKB:Q9HC96",
  "term_id": "GO:0005737",
  "gene_name": "Calpain-10",
  "term_label": "cytoplasm"
}